embryonic pectoral fin morphogenesis [GO:0035118] (biological process) Relationships: is a type of GO:0035113; is a type of GO:0035138 Definition: The process, occurring in the embryo, by which the anatomical structures of the pectoral fin are generated and organized. Pectoral fins are bilaterally paired fins mounted laterally and located behind the gill covers of fish. These fins are used for lateral mobility and propulsion. Sources: GOC:dgh